{
  "term_label": "Unknown biological process",
  "gene_symbol": "NSRP1",
  "gene_name": "Nuclear speckle splicing regulatory protein 1",
  "gene": "UniProtKB:Q9H0G5",
  "term_id": "UNKNOWN:0002"
}